{
  "gene": "UniProtKB:Q6IQ23",
  "term_id": "GO:0005915",
  "term_label": "zonula adherens",
  "gene_name": "Pleckstrin homology domain-containing family A member 7",
  "gene_symbol": "PLEKHA7"
}